{
  "gene_symbol": "SLC35E3",
  "term_label": "transmembrane transport",
  "gene": "UniProtKB:Q7Z769",
  "gene_name": "Solute carrier family 35 member E3",
  "term_id": "GO:0055085"
}